{
  "term_id": "UNKNOWN:0001",
  "gene": "UniProtKB:Q9H1Y0",
  "term_label": "Unknown molecular function",
  "gene_symbol": "ATG5",
  "gene_name": "Autophagy protein 5"
}